regulation of Rho-dependent protein serine/threonine kinase activity [GO:2000298] (BP) Subtypes: GO:2000299 Also known as: regulation of ROCK kinase activity, regulation of Rho-associated protein kinase activity Sources: GOC:mah Definition: Any process that modulates the frequency, rate or extent of Rho-dependent protein serine/threonine kinase activity. Relationships: is a type of regulation of protein serine/threonine kinase activity [GO:0071900]; regulates GO:0072518